acyl-L-homoserine-lactone lactonohydrolase activity [GO:0102007] (molecular function) Definition: Catalysis of the reaction: H2O + an N-acyl-L-homoserine lactone = H+ + an N-acyl-L-homoserine. Sources: EC:3.1.1.81 Relationships: is a type of lactonohydrolase activity [GO:0046573]